{
  "gene_name": "Gap junction gamma-2 protein",
  "term_label": "connexin complex",
  "term_id": "GO:0005922",
  "gene": "UniProtKB:Q5T442",
  "gene_symbol": "GJC2"
}